telomerase inhibitor activity [GO:0010521] (molecular function) Sources: GOC:dph, GOC:krc, GOC:tb Relationships: is a type of GO:0004857; negatively regulates telomerase activity [GO:0003720] Definition: Binds to and stops, prevents or reduces the activity of telomerase.